7,8-didemethyl-8-hydroxy-5-deazariboflavin biosynthetic process [GO:1901852] (biological process) Definition: The chemical reactions and pathways resulting in the formation of 7,8-didemethyl-8-hydroxy-5-deazariboflavin. References: PMID:14593448 Sources: GOC:TermGenie, GOC:yaf, UniPathway:UPA00072 Also known as: 7,8-didemethyl-8-hydroxy-5-deazariboflavin anabolism, 7,8-didemethyl-8-hydroxy-5-deazariboflavin biosynthesis, 7,8-didemethyl-8-hydroxy-5-deazariboflavin formation, 7,8-didemethyl-8-hydroxy-5-deazariboflavin synthesis, coenzyme F0 anabolism, coenzyme F0 biosynthesis, coenzyme F0 biosynthetic process, coenzyme F0 formation, coenzyme F0 synthesis Relationships: is a type of biosynthetic process [GO:0009058]